symbiont-mediated disruption of host mitochondrion [GO:0033659] (biological process) Also known as: disruption by symbiont of host mitochondrion, modification by symbiont of host mitochondrion Relationships: is a type of symbiont-mediated disruption of host cellular anatomical structure [GO:0052008] References: PMID:35069483, PMID:37175745 Sources: GOC:pamgo_curators Definition: The process in which an organism effects a change in the structure or function of host cell mitochondria. The host is defined as the larger of the organisms involved in a symbiotic interaction.